{
  "gene_name": "DNA replication licensing factor MCM6",
  "gene": "UniProtKB:Q14566",
  "term_id": "GO:0042555",
  "term_label": "MCM complex",
  "gene_symbol": "MCM6"
}